establishment of protein localization to membrane [GO:0090150] (BP) Subtypes: protein targeting to membrane [GO:0006612], GO:0032596, protein transport out of plasma membrane raft [GO:0044862], protein import into chloroplast thylakoid membrane [GO:0045038], protein import into peroxisome membrane [GO:0045046], protein insertion into membrane [GO:0051205], establishment of protein localization to plasma membrane [GO:0061951], GO:0090151, GO:0097051, neurotransmitter receptor transport to plasma membrane [GO:0098877], extraction of mislocalized protein from membrane [GO:0140568], establishment of protein localization to postsynaptic membrane [GO:1903540] Also known as: establishment of protein localisation in membrane, establishment of protein localization in membrane Sources: GOC:ascb_2009, GOC:dph, GOC:tb Relationships: is a type of establishment of protein localization [GO:0045184]; is a type of localization within membrane [GO:0051668] Definition: The directed movement of a protein to a specific location in a membrane.